positive regulation of cytoplasmic translational elongation [GO:1900249] (biological process) Also known as: up regulation of cytoplasmic translational elongation, up-regulation of cytoplasmic translational elongation, upregulation of cytoplasmic translational elongation, activation of cytoplasmic translational elongation Definition: Any process that activates or increases the frequency, rate or extent of cytoplasmic translational elongation. Relationships: is_a positive regulation of translational elongation [GO:0045901]; is a type of regulation of cytoplasmic translational elongation [GO:1900247]; positively regulates cytoplasmic translational elongation [GO:0002182] Sources: GOC:TermGenie Subtypes: positive regulation of cytoplasmic translational elongation through polyproline stretches [GO:1903272]